{
  "gene_name": "Gem-associated protein 8",
  "gene": "UniProtKB:Q9NWZ8",
  "term_id": "UNKNOWN:0001",
  "gene_symbol": "GEMIN8",
  "term_label": "Unknown molecular function"
}